keratan sulfate-III proteoglycan biosynthetic process [GO:0140265] (BP) Definition: The chemical reactions and pathways resulting in the formation of keratan sulfate III (KS-III), O-linked via a mannose attached to a serine or a threonine residue in the target protein. References: PMID:29340594 Also known as: O-linked man-keratan sulfate-III proteoglycan biosynthetic process Relationships: is a type of keratan sulfate proteoglycan biosynthetic process [GO:0018146]; is a type of protein O-linked glycosylation via mannose [GO:0035269]